{
  "term_id": "GO:1904071",
  "gene": "UniProtKB:Q9Y6V0",
  "term_label": "presynaptic active zone assembly",
  "gene_symbol": "PCLO",
  "gene_name": "Protein piccolo"
}